{
  "gene": "UniProtKB:Q8N1D5",
  "term_label": "Unknown molecular function",
  "gene_name": "Cilia- and flagella-associated protein 107",
  "term_id": "UNKNOWN:0001",
  "gene_symbol": "CFAP107"
}